{
  "term_id": "GO:0005940",
  "gene_symbol": "SEPTIN4",
  "gene": "UniProtKB:O43236",
  "gene_name": "Septin-4",
  "term_label": "septin ring"
}